{
  "gene": "UniProtKB:P35659",
  "term_label": "histone binding",
  "gene_name": "Protein DEK",
  "gene_symbol": "DEK",
  "term_id": "GO:0042393"
}